asparagine transmembrane import into vacuole [GO:1990591] (biological process) Definition: The directed movement of asparagine into the vacuole across the vacuolar membrane. References: PMID:20388511 Relationships: is a type of amino acid transmembrane import into vacuole [GO:0032975]; is a type of GO:1903713